{
  "gene_name": "Ropporin-1-like protein",
  "term_id": "UNKNOWN:0001",
  "term_label": "Unknown molecular function",
  "gene_symbol": "ROPN1L",
  "gene": "UniProtKB:Q96C74"
}